{
  "term_id": "UNKNOWN:0001",
  "gene_name": "Protein FAM74A4_A6",
  "term_label": "Unknown molecular function",
  "gene": "UniProtKB:Q5TZK3",
  "gene_symbol": "FAM74A6"
}